acrosome assembly [GO:0001675] (biological process) Definition: The formation of the acrosome from the spermatid Golgi. Sources: GOC:dph, GOC:hjd, GOC:tb Also known as: acrosome formation Relationships: is_a developmental process involved in reproduction [GO:0003006]; is a type of GO:0010927; is a type of GO:0022412; is_a GO:0033363; is_a organelle assembly [GO:0070925]; is part of GO:0007286